{
  "term_id": "GO:0055075",
  "gene_name": "Solute carrier family 12 member 1",
  "gene_symbol": "SLC12A1",
  "term_label": "potassium ion homeostasis",
  "gene": "UniProtKB:Q13621"
}